fatty acid derivative transport [GO:1901571] (biological process) Subtypes: diaminopimelate transport [GO:0015830] Relationships: is a type of GO:0006869 Sources: GOC:TermGenie, GOC:pr Definition: The directed movement of a fatty acid derivative into, out of or within a cell, or between cells, by means of some agent such as a transporter or pore.